microbody membrane [GO:0031903] (cellular component) Definition: The lipid bilayer surrounding a microbody. Sources: GOC:mah Relationships: is a type of microbody [GO:0042579]; is_a bounding membrane of organelle [GO:0098588]; is part of microbody [GO:0042579] Subtypes: peroxisomal membrane [GO:0005778]